pyrophosphate-dependent phosphofructokinase complex, alpha-subunit complex [GO:0010317] (cellular component) References: PMID:2170409 Definition: Refers to the alpha subunit of the heterodimeric complex that possesses pyrophosphate-dependent phosphofructokinase activity. Also known as: PFK complex, alpha-subunit Relationships: is a type of catalytic complex [GO:1902494]; is part of pyrophosphate-dependent phosphofructokinase complex [GO:0010316]